{
  "gene": "UniProtKB:Q9NPZ5",
  "term_id": "GO:0005975",
  "gene_name": "Galactosylgalactosylxylosylprotein 3-beta-glucuronosyltransferase 2",
  "term_label": "carbohydrate metabolic process",
  "gene_symbol": "B3GAT2"
}